{
  "gene_symbol": "SEMA4D",
  "term_label": "axon guidance",
  "gene_name": "Semaphorin-4D",
  "term_id": "GO:0007411",
  "gene": "UniProtKB:Q92854"
}